{
  "gene_symbol": "KRTAP9-9",
  "gene_name": "Keratin-associated protein 9-9",
  "term_label": "Unknown cellular component",
  "gene": "UniProtKB:Q9BYP9",
  "term_id": "UNKNOWN:0003"
}